{
  "term_label": "Unknown biological process",
  "gene": "UniProtKB:Q5TAG4",
  "gene_name": "Neuroblastoma breakpoint family member 12",
  "term_id": "UNKNOWN:0002",
  "gene_symbol": "NBPF12"
}